{
  "gene": "UniProtKB:O14818",
  "gene_name": "Proteasome subunit alpha type-7",
  "term_label": "proteasome-mediated ubiquitin-dependent protein catabolic process",
  "term_id": "GO:0043161",
  "gene_symbol": "PSMA7"
}